{
  "term_id": "GO:0000776",
  "gene_name": "Anaphase-promoting complex subunit 16",
  "gene": "UniProtKB:Q96DE5",
  "term_label": "kinetochore",
  "gene_symbol": "ANAPC16"
}